{
  "term_id": "UNKNOWN:0002",
  "term_label": "Unknown biological process",
  "gene_symbol": "TRBJ2-6",
  "gene": "UniProtKB:A0A0A0MT70",
  "gene_name": "T cell receptor beta joining 2-6"
}